purine-specific nucleoside:sodium symporter activity [GO:0015390] (molecular function) Definition: Enables the transfer of a solute or solutes from one side of a membrane to the other according to the reaction: purine(out) + Na+(out) = nucleoside(in) + Na+(in). Sources: TC:2.A.41.2.1 Relationships: is a type of solute:sodium symporter activity [GO:0015370]